hibernation [GO:0042750] (biological process) Relationships: is a type of dormancy process [GO:0022611] References: PMID:1945046 Sources: GOC:jl Definition: Any process in which an organism enters and maintains a period of dormancy in which to pass the winter. It is characterized by narcosis and by sharp reduction in body temperature and metabolic activity and by a depression of vital signs.